U2AF complex [GO:0089701] (CC) Also known as: U2 accessory factor, U2AF Definition: A heterodimeric protein complex consisting of conserved large and small U2AF subunits that contributes to spliceosomal RNA splicing by binding to consensus sequences at the 3' splice site. U2AF is required to stabilize the association of the U2 snRNP with the branch point. Relationships: is a type of GO:0140513 References: PMID:15231733, PMID:1538748, PMID:2963698, PMID:8657565 Sources: GOC:dos, GOC:mah